dibenzothiophene dihydrodiol dehydrogenase activity [GO:0018513] (molecular function) Also known as: cis-1,2-dihydroxy-1,2-dihydrodibenzothiophene:NAD+ oxidoreductase activity Sources: EC:1.3.1.60, RHEA:24188 Definition: Catalysis of the reaction: cis-1,2-dihydroxy-1,2-dihydrodibenzothiophene + NAD+ = 1,2-dihydroxydibenzothiophene + H+ + NADH. Relationships: is a type of GO:0016628